{
  "gene_name": "HLA class II histocompatibility antigen, DQ alpha 1 chain",
  "gene_symbol": "HLA-DQA1",
  "gene": "UniProtKB:P01909",
  "term_id": "GO:0050870",
  "term_label": "positive regulation of T cell activation"
}